{
  "gene_symbol": "MEAK7",
  "term_id": "GO:0005634",
  "term_label": "nucleus",
  "gene_name": "MTOR-associated protein MEAK7",
  "gene": "UniProtKB:Q6P9B6"
}